{
  "gene_name": "ADP-ribosylation factor-like protein 9",
  "gene_symbol": "ARL9",
  "term_id": "UNKNOWN:0002",
  "term_label": "Unknown biological process",
  "gene": "UniProtKB:Q6T311"
}